{
  "gene_symbol": "CDKL3",
  "term_label": "positive regulation of dendrite morphogenesis",
  "gene": "UniProtKB:Q8IVW4",
  "term_id": "GO:0050775",
  "gene_name": "Cyclin-dependent kinase-like 3"
}